{
  "term_id": "GO:0005096",
  "gene_name": "TBC1 domain family member 30",
  "gene": "UniProtKB:Q9Y2I9",
  "term_label": "GTPase activator activity",
  "gene_symbol": "TBC1D30"
}